{
  "term_label": "nuclear pore",
  "gene_name": "mRNA export factor RAE1",
  "gene_symbol": "RAE1",
  "gene": "UniProtKB:P78406",
  "term_id": "GO:0005643"
}